{
  "term_label": "nucleus",
  "gene_symbol": "KNL1",
  "gene_name": "Kinetochore scaffold 1",
  "gene": "UniProtKB:Q8NG31",
  "term_id": "GO:0005634"
}